cell pole [GO:0060187] (cellular component) Subtypes: apical pole of neuron [GO:0044225], basal pole of neuron [GO:0044226], cell tip [GO:0051286], basal pole of outer hair cell [GO:0090712], GO:1990901, new cell pole [GO:1990902] Relationships: is a type of cellular anatomical structure [GO:0110165] Sources: GOC:dph Note: Note that this term differs from 'cell tip ; GO:0051286' in that it is applicable to a broad range of cell shapes including spherical and cuboidal. Definition: Either of two different areas at opposite ends of an axis of a cell.